regulation of cell diameter [GO:0060305] (biological process) Sources: GOC:dph, GOC:tb Definition: Any process that modulates the diameter of a cell, the length of a line segment that crosses through the center of a circular section through a cell. Relationships: is a type of regulation of cell size [GO:0008361] Also known as: regulation of cell width